{
  "gene_symbol": "PRORSD1P",
  "term_label": "Unknown biological process",
  "gene_name": "Putative prolyl-tRNA synthetase associated domain-containing protein 1",
  "term_id": "UNKNOWN:0002",
  "gene": "UniProtKB:A6NEY8"
}